detection of endoplasmic reticulum overloading [GO:0002234] (biological process) Definition: The series of events in which a stimulus generated by the accumulation of normal or misfolded proteins in the endoplasmic reticulum is received and converted into a molecular signal. References: PMID:10390516 Sources: GOC:add Also known as: detection of ER overloading Relationships: is a type of ER overload response [GO:0006983]; is a type of GO:0009595